regulation of somatic stem cell population maintenance [GO:1904672] (biological process) References: PMID:19409607 Sources: GOC:BHF, GOC:BHF_miRNA, GOC:TermGenie, GOC:rph, GO_REF:0000058 Relationships: is a type of regulation of stem cell population maintenance [GO:2000036]; regulates somatic stem cell population maintenance [GO:0035019] Definition: Any process that modulates the frequency, rate or extent of somatic stem cell population maintenance. Subtypes: regulation of mesenchymal cell apoptotic process involved in nephron morphogenesis [GO:0072039], GO:1904673, positive regulation of somatic stem cell population maintenance [GO:1904674]